{
  "term_label": "Unknown molecular function",
  "gene_name": "SH3 domain-binding protein 2",
  "term_id": "UNKNOWN:0001",
  "gene_symbol": "SH3BP2",
  "gene": "UniProtKB:P78314"
}